{
  "term_id": "GO:0005737",
  "gene_name": "Dynamin-binding protein",
  "term_label": "cytoplasm",
  "gene": "UniProtKB:Q6XZF7",
  "gene_symbol": "DNMBP"
}